{
  "gene_name": "CKLF-like MARVEL transmembrane domain-containing protein 5",
  "gene_symbol": "CMTM5",
  "gene": "UniProtKB:Q96DZ9",
  "term_label": "Unknown biological process",
  "term_id": "UNKNOWN:0002"
}